polyketide biosynthetic process [GO:0030639] (biological process) Definition: The chemical reactions and pathways resulting in the formation of polyketides, any of a diverse group of natural products synthesized via linear poly-beta-ketones, which are themselves formed by repetitive head-to-tail addition of acetyl (or substituted acetyl) units indirectly derived from acetate (or a substituted acetate) by a mechanism similar to that for fatty acid biosynthesis but without the intermediate reductive steps. Sources: GOC:mah, ISBN:0198506732 Also known as: polyketide anabolism, polyketide biosynthesis, polyketide formation, polyketide synthesis Relationships: is a type of GO:0030638; is_a secondary metabolite biosynthetic process [GO:0044550] Subtypes: GO:0033068, ansamycin biosynthetic process [GO:0033070], tetracycline biosynthetic process [GO:0043644], GO:0140446, 1,8-dihydroxynaphthalene-melanin biosynthetic process [GO:0140614], mycophenolic acid biosynthetic process [GO:0140722], patulin biosynthetic process [GO:0140723], lovastatin biosynthetic process [GO:0140735], ilicicolin H biosynthetic process [GO:0140781], GO:0140783, GO:0140872, mevastatin biosynthetic process [GO:0140877], asperfuranone biosynthetic process [GO:1900554], F-9775A biosynthetic process [GO:1900611], F-9775B biosynthetic process [GO:1900614], averantin biosynthetic process [GO:1900763], fonsecin biosynthetic process [GO:1900769], tetracenomycin C biosynthetic process [GO:1901106], granaticin biosynthetic process [GO:1901109], aspyridone A biosynthetic process [GO:1901518], GO:1901521, olivetolic acid biosynthetic process [GO:1901697], oxytetracycline biosynthetic process [GO:1901763], daunorubicin biosynthetic process [GO:1901771], neosartoricin biosynthetic process [GO:1902050] Regulation: regulated by regulation of polyketide biosynthetic process [GO:1900732]; negatively regulated by negative regulation of polyketide biosynthetic process [GO:1900733]; positively regulated by positive regulation of polyketide biosynthetic process [GO:1900734]